{
  "term_label": "Unknown cellular component",
  "gene": "UniProtKB:Q9BY79",
  "gene_name": "Membrane frizzled-related protein",
  "term_id": "UNKNOWN:0003",
  "gene_symbol": "MFRP"
}